10-hydroxytaxane O-acetyltransferase activity [GO:0050639] (MF) Also known as: acetyl-CoA:taxan-10beta-ol O-acetyltransferase, acetyl coenzyme A: 10-hydroxytaxane O-acetyltransferase activity, acetyl coenzyme A:10-hydroxytaxane O-acetyltransferase activity Sources: EC:2.3.1.163, RHEA:18837 Relationships: is a type of O-acetyltransferase activity [GO:0016413] Definition: Catalysis of the reaction: 10-desacetyltaxuyunnanin C + acetyl-CoA = CoA + taxuyunnanin C.